{
  "gene_symbol": "PSMB3",
  "gene": "UniProtKB:P49720",
  "term_id": "GO:0043161",
  "gene_name": "Proteasome subunit beta type-3",
  "term_label": "proteasome-mediated ubiquitin-dependent protein catabolic process"
}